{
  "gene_name": "Probable tRNA methyltransferase 9B",
  "gene": "UniProtKB:Q9P272",
  "gene_symbol": "TRMT9B",
  "term_label": "nucleus",
  "term_id": "GO:0005634"
}